{
  "term_label": "neuron differentiation",
  "term_id": "GO:0030182",
  "gene_name": "Iroquois-class homeodomain protein IRX-1",
  "gene": "UniProtKB:P78414",
  "gene_symbol": "IRX1"
}